{
  "gene_name": "Protein FAM104B",
  "term_id": "UNKNOWN:0003",
  "term_label": "Unknown cellular component",
  "gene": "UniProtKB:Q5XKR9",
  "gene_symbol": "FAM104B"
}